{
  "gene_name": "Histone PARylation factor 1",
  "gene": "UniProtKB:Q9NWY4",
  "term_id": "GO:0072572",
  "term_label": "poly-ADP-D-ribose binding",
  "gene_symbol": "HPF1"
}